{
  "term_id": "UNKNOWN:0001",
  "gene_symbol": "NBPF19",
  "gene_name": "Neuroblastoma breakpoint family member 19",
  "gene": "UniProtKB:A0A087WUL8",
  "term_label": "Unknown molecular function"
}